{
  "term_label": "Unknown molecular function",
  "gene_symbol": "PHF23",
  "gene": "UniProtKB:Q9BUL5",
  "gene_name": "PHD finger protein 23",
  "term_id": "UNKNOWN:0001"
}